positive regulation of vascular associated smooth muscle cell apoptotic process [GO:1905461] (biological process) Also known as: positive regulation of VSMC apoptotic process, positive regulation of vascular smooth muscle cell apoptotic process, up regulation of VSMC apoptotic process, up regulation of vascular associated smooth muscle cell apoptotic process, up regulation of vascular smooth muscle cell apoptotic process, up-regulation of VSMC apoptotic process, up-regulation of vascular associated smooth muscle cell apoptotic process, up-regulation of vascular smooth muscle cell apoptotic process, upregulation of VSMC apoptotic process, upregulation of vascular associated smooth muscle cell apoptotic process, upregulation of vascular smooth muscle cell apoptotic process, activation of VSMC apoptosis, activation of VSMC apoptotic process, activation of vascular associated smooth muscle cell apoptosis, activation of vascular associated smooth muscle cell apoptotic process, activation of vascular smooth muscle cell apoptosis, activation of vascular smooth muscle cell apoptotic process, positive regulation of VSMC apoptosis, positive regulation of vascular associated smooth muscle cell apoptosis, positive regulation of vascular smooth muscle cell apoptosis, up regulation of VSMC apoptosis, up regulation of vascular associated smooth muscle cell apoptosis, up regulation of vascular smooth muscle cell apoptosis, up-regulation of VSMC apoptosis, up-regulation of vascular associated smooth muscle cell apoptosis, up-regulation of vascular smooth muscle cell apoptosis, upregulation of VSMC apoptosis, upregulation of vascular associated smooth muscle cell apoptosis, upregulation of vascular smooth muscle cell apoptosis Definition: Any process that activates or increases the frequency, rate or extent of vascular associated smooth muscle cell apoptotic process. Relationships: is a type of positive regulation of smooth muscle cell apoptotic process [GO:0034393]; is a type of regulation of vascular associated smooth muscle cell apoptotic process [GO:1905459]; positively regulates vascular associated smooth muscle cell apoptotic process [GO:1905288] References: PMID:26493107 Sources: GOC:BHF, GOC:BHF_miRNA, GOC:TermGenie, GOC:rph, GO_REF:0000058